{
  "term_label": "immunoglobulin complex",
  "gene_symbol": "TRAV9-1",
  "term_id": "GO:0019814",
  "gene_name": "T cell receptor alpha variable 9-1",
  "gene": "UniProtKB:A0A075B6T8"
}